{
  "gene": "UniProtKB:O95394",
  "gene_name": "Phosphoacetylglucosamine mutase",
  "gene_symbol": "PGM3",
  "term_label": "hemopoiesis",
  "term_id": "GO:0030097"
}